{
  "gene": "UniProtKB:Q8TD86",
  "term_id": "GO:0000226",
  "gene_symbol": "CALML6",
  "gene_name": "Calmodulin-like protein 6",
  "term_label": "microtubule cytoskeleton organization"
}